copal-8-ol diphosphate(3-) catabolic process [GO:1902242] (biological process) Definition: The chemical reactions and pathways resulting in the breakdown of copal-8-ol diphosphate(3-). Also known as: copal-8-ol diphosphate(3-) breakdown, copal-8-ol diphosphate(3-) catabolism, copal-8-ol diphosphate(3-) degradation Relationships: is a type of phospholipid catabolic process [GO:0009395]; is a type of diterpenoid catabolic process [GO:0016103] References: PMID:22672125 Sources: GOC:TermGenie